{
  "gene_name": "Large ribosomal subunit protein bL20m",
  "gene_symbol": "MRPL20",
  "term_id": "UNKNOWN:0002",
  "gene": "UniProtKB:Q9BYC9",
  "term_label": "Unknown biological process"
}